{
  "term_id": "GO:0005654",
  "gene_name": "Spindlin-2A",
  "term_label": "nucleoplasm",
  "gene": "UniProtKB:Q99865",
  "gene_symbol": "SPIN2A"
}